{
  "term_id": "GO:0003341",
  "gene": "UniProtKB:Q5T0N1",
  "term_label": "cilium movement",
  "gene_symbol": "CFAP70",
  "gene_name": "Cilia- and flagella-associated protein 70"
}